{
  "term_id": "GO:0005829",
  "gene_name": "Cellular retinoic acid-binding protein 2",
  "term_label": "cytosol",
  "gene_symbol": "CRABP2",
  "gene": "UniProtKB:P29373"
}